{
  "term_id": "GO:0008420",
  "term_label": "RNA polymerase II CTD heptapeptide repeat phosphatase activity",
  "gene": "UniProtKB:A0A1W2PQD8",
  "gene_symbol": "SSU72L2",
  "gene_name": "RNA polymerase II subunit A C-terminal domain phosphatase SSU72 like protein 2"
}